{
  "gene": "UniProtKB:Q9H4B6",
  "gene_name": "Protein salvador homolog 1",
  "term_label": "Unknown molecular function",
  "gene_symbol": "SAV1",
  "term_id": "UNKNOWN:0001"
}